{
  "gene_symbol": "SPAG4",
  "term_label": "meiotic nuclear membrane microtubule tethering complex",
  "gene": "UniProtKB:Q9NPE6",
  "term_id": "GO:0034993",
  "gene_name": "Sperm-associated antigen 4 protein"
}